{
  "gene_name": "Olfactory receptor 5H14",
  "gene": "UniProtKB:A6NHG9",
  "term_label": "Unknown biological process",
  "gene_symbol": "OR5H14",
  "term_id": "UNKNOWN:0002"
}